{
  "gene_symbol": "TPM4",
  "gene_name": "Tropomyosin alpha-4 chain",
  "term_id": "GO:0051015",
  "gene": "UniProtKB:P67936",
  "term_label": "actin filament binding"
}